deep nuclear neuron precursor proliferation [GO:0021927] (biological process) Relationships: is a type of GO:0021923 Definition: The multiplication or reproduction of neuroblasts that will give rise to deep nuclear neurons. References: PMID:15157725 Sources: GOC:cls, GOC:dgh, GOC:dph, GOC:jid, GO_REF:0000021